{
  "term_id": "GO:0045296",
  "gene_symbol": "PTPRO",
  "gene": "UniProtKB:Q16827",
  "gene_name": "Receptor-type tyrosine-protein phosphatase O",
  "term_label": "cadherin binding"
}